{
  "term_id": "GO:0043235",
  "gene_name": "Granulocyte colony-stimulating factor receptor",
  "gene_symbol": "CSF3R",
  "term_label": "receptor complex",
  "gene": "UniProtKB:Q99062"
}